{
  "term_id": "GO:0005615",
  "gene_name": "Adipolin",
  "gene_symbol": "C1QTNF12",
  "term_label": "extracellular space",
  "gene": "UniProtKB:Q5T7M4"
}